{
  "gene_name": "Serine_threonine-protein kinase tousled-like 2",
  "gene_symbol": "TLK2",
  "term_label": "intracellular signal transduction",
  "gene": "UniProtKB:Q86UE8",
  "term_id": "GO:0035556"
}